{
  "gene": "UniProtKB:P56693",
  "term_id": "GO:0002009",
  "gene_symbol": "SOX10",
  "gene_name": "Transcription factor SOX-10",
  "term_label": "morphogenesis of an epithelium"
}